corticosterone binding [GO:1903875] (molecular function) Definition: Binding to corticosterone. References: PMID:10802282 Sources: GOC:TermGenie, GOC:mr, GO_REF:0000067 Relationships: is a type of GO:0043178; is a type of steroid hormone binding [GO:1990239]